{
  "gene_symbol": "CAVIN2",
  "gene": "UniProtKB:O95810",
  "gene_name": "Caveolae-associated protein 2",
  "term_id": "GO:0005901",
  "term_label": "caveola"
}